{
  "term_label": "DNA-binding transcription factor activity, RNA polymerase II-specific",
  "gene_name": "Zinc finger protein 595",
  "term_id": "GO:0000981",
  "gene": "UniProtKB:Q8IYB9",
  "gene_symbol": "ZNF595"
}